regulation of dense core granule biogenesis [GO:2000705] (biological process) Sources: GOC:obol Relationships: is_a regulation of cellular component biogenesis [GO:0044087]; regulates dense core granule biogenesis [GO:0061110] Definition: Any process that modulates the frequency, rate or extent of dense core granule biogenesis. Subtypes: negative regulation of dense core granule biogenesis [GO:2000706], positive regulation of dense core granule biogenesis [GO:2000707]